{
  "term_label": "nuclear envelope",
  "term_id": "GO:0005635",
  "gene_name": "Nuclear envelope integral membrane protein 2",
  "gene_symbol": "NEMP2",
  "gene": "UniProtKB:A6NFY4"
}